{
  "gene_symbol": "LINC01619",
  "gene_name": "Uncharacterized protein encoded by LINC01619",
  "gene": "UniProtKB:G3V211",
  "term_label": "Unknown cellular component",
  "term_id": "UNKNOWN:0003"
}